{
  "gene_symbol": "ZNF221",
  "term_id": "UNKNOWN:0003",
  "gene_name": "Zinc finger protein 221",
  "gene": "UniProtKB:Q9UK13",
  "term_label": "Unknown cellular component"
}